{
  "term_label": "alpha2-adrenergic receptor activity",
  "term_id": "GO:0004938",
  "gene": "UniProtKB:P18089",
  "gene_name": "Alpha-2B adrenergic receptor",
  "gene_symbol": "ADRA2B"
}